MAML2-RBP-Jkappa-ICN3 complex [GO:0071177] (cellular component) References: PMID:12370315 Definition: A protein complex that consists of the intracellular domain of Notch3 (ICN3), the DNA-binding transcription factor RBP-Jkappa, and the transcriptional coactivator Mastermind-like-2 (MAML2); the complex is involved in transcriptional activation in response to Notch-mediated signaling. Relationships: is_a nuclear protein-containing complex [GO:0140513] Also known as: MAML2-RBP-Jkappa-Notch3 complex